telencephalon glial cell migration [GO:0022030] (biological process) Sources: GOC:cls, GOC:dgh, GOC:dph, GOC:jid, GO_REF:0000021 Definition: The orderly movement of glial cells through the telencephalon. Relationships: is a type of glial cell migration [GO:0008347]; is a type of telencephalon cell migration [GO:0022029] Subtypes: GO:0021801, oligodendrocyte cell migration from the subpallium to the cortex [GO:0021829], telencephalon astrocyte cell migration [GO:0022031], telencephalon oligodendrocyte cell migration [GO:0022032], telencephalon microglial cell migration [GO:0022033]